negative regulation of mitotic sister chromatid arm separation [GO:1905823] (biological process) Definition: Any process that stops, prevents or reduces the frequency, rate or extent of mitotic sister chromatid arm separation. References: PMID:18765790 Sources: GOC:TermGenie, GOC:als, GO_REF:0000058 Relationships: is_a regulation of mitotic sister chromatid arm separation [GO:1905822]; is a type of negative regulation of mitotic sister chromatid separation [GO:2000816]; negatively regulates mitotic sister chromatid arm separation [GO:1990891] Also known as: down regulation of mitotic sister chromatid arm separation, down-regulation of mitotic sister chromatid arm separation, downregulation of mitotic sister chromatid arm separation, inhibition of mitotic sister chromatid arm separation